dinoflagellate sulcus [GO:0097612] (cellular component) Relationships: is a type of cell surface furrow [GO:0097610] Note: The term name refers to a taxonomic group to make the label unique with respect to similarly-named anatomical structures. Also, the ventral (front) side of a dinoflagellate cell is the one where the sulcus is located (as opposed to the dorsal (back) side). Definition: A cell surface furrow that occurs on the ventral side of a dinoflagellate cell. It partially houses the longitudinal flagellum. The sulcus intersects with the cingulum on the ventral side of a dinoflagellate cell. Also known as: sulcus, longitudinal furrow, longitudinal groove Subtypes: dinoflagellate sulcal notch [GO:0097618] References: PMID:20561119 Sources: GOC:at, Wikipedia:Dinoflagellate#Morphology, http://tolweb.org/Dinoflagellates/2445